{
  "term_id": "GO:0003714",
  "gene_name": "Zinc finger protein ZFPM2",
  "term_label": "transcription corepressor activity",
  "gene": "UniProtKB:Q8WW38",
  "gene_symbol": "ZFPM2"
}